{
  "gene": "UniProtKB:Q9BZM1",
  "gene_symbol": "PLA2G12A",
  "gene_name": "Group XIIA secretory phospholipase A2",
  "term_label": "Unknown biological process",
  "term_id": "UNKNOWN:0002"
}